nuclear receptor binding [GO:0016922] (molecular function) Subtypes: nuclear estrogen receptor binding [GO:0030331], nuclear mineralocorticoid receptor binding [GO:0031962], nuclear progesterone receptor binding [GO:0033142], nuclear glucocorticoid receptor binding [GO:0035259], GO:0042809, nuclear retinoic acid receptor binding [GO:0042974], nuclear thyroid hormone receptor binding [GO:0046966], GO:0050681 Relationships: is a type of RNA polymerase II-specific DNA-binding transcription factor binding [GO:0061629] References: PMID:7776974 Also known as: steroid hormone receptor binding, ligand-dependent nuclear receptor binding, nuclear hormone receptor binding, ligand-dependent nuclear receptor interactor activity Definition: Binding to a nuclear receptor protein. Nuclear receptor proteins are DNA-binding transcription factors which are regulated by binding to a ligand.